{
  "gene_symbol": "LILRB2",
  "gene": "UniProtKB:Q8N423",
  "term_id": "GO:0140105",
  "gene_name": "Leukocyte immunoglobulin-like receptor subfamily B member 2",
  "term_label": "interleukin-10-mediated signaling pathway"
}